{
  "term_id": "GO:0000785",
  "gene": "UniProtKB:O00273",
  "gene_name": "DNA fragmentation factor subunit alpha",
  "term_label": "chromatin",
  "gene_symbol": "DFFA"
}